{
  "gene": "UniProtKB:P17098",
  "term_label": "negative regulation of transcription by RNA polymerase II",
  "gene_symbol": "ZNF8",
  "term_id": "GO:0000122",
  "gene_name": "Zinc finger protein 8"
}